RNA guanosine insertion [GO:0070709] (biological process) Sources: GOC:cb, GOC:mah Relationships: is a type of RNA nucleotide insertion [GO:0070705] Definition: The modification of an RNA molecule by insertion of a guanosine nucleotide. Also known as: RNA G insertion